extracellularly glycine-gated ion channel activity [GO:0016933] (molecular function) Subtypes: extracellularly glycine-gated chloride channel activity [GO:0016934] Relationships: is a type of excitatory extracellular ligand-gated monoatomic ion channel activity [GO:0005231] Also known as: glycine receptor, extracellular-glycine-gated ion channel activity Sources: GOC:mtg_transport, ISBN:0815340729 Definition: Enables the transmembrane transfer of an ion by a channel that opens when glycine is bound by the channel complex or one of its constituent parts on the extracellular side of the plasma membrane.